{
  "term_id": "GO:0005096",
  "gene_symbol": "DLC1",
  "term_label": "GTPase activator activity",
  "gene": "UniProtKB:Q96QB1",
  "gene_name": "Rho GTPase-activating protein 7"
}